{
  "term_id": "GO:0141014",
  "term_label": "ribosome hibernation",
  "gene_name": "Death-associated protein 1",
  "gene": "UniProtKB:P51397",
  "gene_symbol": "DAP"
}